{
  "term_id": "GO:0035097",
  "gene": "UniProtKB:Q14686",
  "gene_symbol": "NCOA6",
  "gene_name": "Nuclear receptor coactivator 6",
  "term_label": "histone methyltransferase complex"
}